{
  "gene_symbol": "DUSP7",
  "term_id": "GO:0070373",
  "gene": "UniProtKB:Q16829",
  "gene_name": "Dual specificity protein phosphatase 7",
  "term_label": "negative regulation of ERK1 and ERK2 cascade"
}